{
  "term_label": "cytoplasm",
  "gene": "UniProtKB:Q6ZVD8",
  "term_id": "GO:0005737",
  "gene_name": "PH domain leucine-rich repeat-containing protein phosphatase 2",
  "gene_symbol": "PHLPP2"
}